cAMP response element binding [GO:0035497] (MF) References: PMID:2875459, PMID:2900470 Definition: Binding to a cyclic AMP response element (CRE), a short palindrome-containing sequence found in the promoters of genes whose expression is regulated in response to cyclic AMP. Relationships: is_a RNA polymerase II cis-regulatory region sequence-specific DNA binding [GO:0000978] Also known as: CRE binding, cAMP-responsive element binding, cyclic AMP response element binding, cyclic-AMP response element binding, cyclic-AMP-responsive element binding